{
  "gene_symbol": "RPRML",
  "term_label": "Unknown biological process",
  "term_id": "UNKNOWN:0002",
  "gene": "UniProtKB:Q8N4K4",
  "gene_name": "Reprimo-like protein"
}